{
  "term_id": "UNKNOWN:0002",
  "gene": "UniProtKB:A8MZ97",
  "term_label": "Unknown biological process",
  "gene_name": "Uncharacterized protein C2orf74",
  "gene_symbol": "C2orf74"
}